{
  "gene_name": "Putative protein T-ENOL",
  "term_id": "UNKNOWN:0001",
  "term_label": "Unknown molecular function",
  "gene": "UniProtKB:P0DO92",
  "gene_symbol": "CDIPTOSP"
}